{
  "gene_name": "Merlin",
  "gene_symbol": "NF2",
  "term_label": "adherens junction",
  "gene": "UniProtKB:P35240",
  "term_id": "GO:0005912"
}